{
  "term_id": "GO:0000978",
  "gene_name": "Zinc finger protein Gfi-1b",
  "gene": "UniProtKB:Q5VTD9",
  "gene_symbol": "GFI1B",
  "term_label": "RNA polymerase II cis-regulatory region sequence-specific DNA binding"
}